{
  "gene": "UniProtKB:O95425",
  "gene_symbol": "SVIL",
  "term_id": "GO:0015629",
  "gene_name": "Supervillin",
  "term_label": "actin cytoskeleton"
}